{
  "term_id": "GO:0000981",
  "gene_name": "Zinc finger protein 280D",
  "gene": "UniProtKB:Q6N043",
  "term_label": "DNA-binding transcription factor activity, RNA polymerase II-specific",
  "gene_symbol": "ZNF280D"
}